{
  "term_id": "UNKNOWN:0002",
  "term_label": "Unknown biological process",
  "gene_symbol": "INPP1",
  "gene": "UniProtKB:P49441",
  "gene_name": "Inositol polyphosphate 1-phosphatase"
}